5'-flap-structured DNA binding [GO:0070338] (molecular function) Definition: Binding to a 5'-flap structure in DNA. A DNA flap structure is one in which a single-stranded 5'-end of DNA or RNA protrudes from a double-stranded DNA molecule. 5'-flap structures can be formed during DNA repair or lagging strand synthesis; in the latter case RNA flaps form from lagging strand RNA primers. References: PMID:15189154 Sources: GOC:mah Relationships: is a type of flap-structured DNA binding [GO:0070336]